{
  "term_label": "membrane",
  "gene_name": "Putative taste receptor type 2 member 33",
  "term_id": "GO:0016020",
  "gene_symbol": "TAS2R33",
  "gene": "UniProtKB:P0DSN6"
}